{
  "gene_symbol": "TRIP12",
  "gene_name": "E3 ubiquitin-protein ligase TRIP12",
  "gene": "UniProtKB:Q14669",
  "term_id": "GO:0016607",
  "term_label": "nuclear speck"
}